regulation of neural crest formation [GO:0090299] (biological process) Relationships: is a type of regulation of epithelial to mesenchymal transition [GO:0010717]; is a type of regulation of anatomical structure morphogenesis [GO:0022603]; RO_0002211 GO:0014029 Definition: Any process that modulates the rate, frequency, or extent of neural crest formation. Neural crest formation is the formation of the specialized region of ectoderm between the neural ectoderm (neural plate) and non-neural ectoderm. The neural crest gives rise to the neural crest cells that migrate away from this region as neural tube formation proceeds. Sources: GOC:tb Subtypes: positive regulation of neural crest formation [GO:0090300], negative regulation of neural crest formation [GO:0090301], regulation of neural crest cell fate specification [GO:1905295]